{
  "term_id": "UNKNOWN:0002",
  "term_label": "Unknown biological process",
  "gene": "UniProtKB:Q86UK5",
  "gene_name": "Limbin",
  "gene_symbol": "EVC2"
}